{
  "term_label": "regulation of transcription by RNA polymerase II",
  "gene_name": "Forkhead box protein D4-like 5",
  "term_id": "GO:0006357",
  "gene_symbol": "FOXD4L5",
  "gene": "UniProtKB:Q5VV16"
}